carbon dioxide transmembrane transporter activity [GO:0035379] (molecular function) Definition: Enables the transfer of carbon dioxide (CO2) from one side of a membrane to the other. Sources: GOC:yaf Relationships: is a type of transmembrane transporter activity [GO:0022857]; is part of GO:0035378